{
  "term_label": "type II transforming growth factor beta receptor binding",
  "gene_name": "Transforming growth factor beta receptor type 3",
  "gene_symbol": "TGFBR3",
  "gene": "UniProtKB:Q03167",
  "term_id": "GO:0005114"
}